regulation of stress-activated protein kinase signaling cascade [GO:0070302] (biological process) Subtypes: regulation of stress-activated MAPK cascade [GO:0032872], negative regulation of stress-activated protein kinase signaling cascade [GO:0070303], positive regulation of stress-activated protein kinase signaling cascade [GO:0070304] Also known as: regulation of SAPK signaling pathway, regulation of stress-activated protein kinase signaling pathway, regulation of stress-activated protein kinase signalling pathway Sources: GOC:mah Relationships: is a type of regulation of cellular response to stress [GO:0080135]; is a type of regulation of intracellular signal transduction [GO:1902531]; regulates stress-activated protein kinase signaling cascade [GO:0031098] Definition: Any process that modulates the frequency, rate or extent of signaling via a stress-activated protein kinase signaling cascade.